{
  "gene": "UniProtKB:P06744",
  "gene_name": "Glucose-6-phosphate isomerase",
  "term_label": "glucose-6-phosphate isomerase activity",
  "term_id": "GO:0004347",
  "gene_symbol": "GPI"
}